{
  "gene_name": "PWWP domain-containing DNA repair factor 3B",
  "term_id": "UNKNOWN:0003",
  "gene": "UniProtKB:Q5H9M0",
  "term_label": "Unknown cellular component",
  "gene_symbol": "PWWP3B"
}